{
  "gene": "UniProtKB:P54707",
  "term_label": "intracellular potassium ion homeostasis",
  "gene_name": "Potassium-transporting ATPase alpha chain 2",
  "gene_symbol": "ATP12A",
  "term_id": "GO:0030007"
}